choloylglycine hydrolase activity [GO:0045302] (MF) Sources: EC:3.5.1.24 Also known as: 3alpha,7alpha,12alpha-trihydroxy-5beta-cholan-24-oylglycine amidohydrolase activity, bile salt hydrolase activity, choloyltaurine hydrolase activity, glycocholase activity Relationships: is a type of hydrolase activity, acting on carbon-nitrogen (but not peptide) bonds, in linear amides [GO:0016811] Definition: Catalysis of the reaction: 3-alpha,7-alpha,12-alpha-trihydroxy-5-beta-cholan-24-oylglycine + H2O = 3-alpha,7-alpha,12-alpha-trihydroxy-5-beta-cholanate + glycine.